{
  "term_id": "GO:0005739",
  "gene_symbol": "OXCT1",
  "gene_name": "Succinyl-CoA:3-ketoacid coenzyme A transferase 1, mitochondrial",
  "term_label": "mitochondrion",
  "gene": "UniProtKB:P55809"
}